{
  "term_label": "GABA-A receptor activity",
  "gene_name": "Gamma-aminobutyric acid receptor subunit alpha-4",
  "gene": "UniProtKB:P48169",
  "term_id": "GO:0004890",
  "gene_symbol": "GABRA4"
}